{
  "gene_name": "Glycine receptor subunit alpha-2",
  "term_id": "UNKNOWN:0003",
  "gene": "UniProtKB:P23416",
  "gene_symbol": "GLRA2",
  "term_label": "Unknown cellular component"
}